{
  "term_id": "GO:0005743",
  "term_label": "mitochondrial inner membrane",
  "gene_name": "m-AAA protease-interacting protein 1, mitochondrial",
  "gene": "UniProtKB:Q8WWC4",
  "gene_symbol": "MAIP1"
}